positive regulation of BMP secretion [GO:1900144] (biological process) Definition: Any process that activates or increases the frequency, rate or extent of BMP secretion. Sources: GOC:TermGenie, GOC:sart Also known as: positive regulation of BMP protein secretion, positive regulation of bone morphogenetic protein secretion, up regulation of BMP protein secretion, up regulation of BMP secretion, up regulation of bone morphogenetic protein secretion, up-regulation of BMP protein secretion, up-regulation of BMP secretion, up-regulation of bone morphogenetic protein secretion, upregulation of BMP protein secretion, upregulation of BMP secretion, upregulation of bone morphogenetic protein secretion, activation of BMP protein secretion, activation of BMP secretion, activation of bone morphogenetic protein secretion Relationships: is a type of positive regulation of cell communication [GO:0010647]; is a type of positive regulation of signaling [GO:0023056]; is a type of positive regulation of protein secretion [GO:0050714]; is a type of GO:2001284; positively regulates BMP secretion [GO:0038055]